{
  "gene_name": "Protein S100-A5",
  "term_label": "calcium-dependent protein binding",
  "gene_symbol": "S100A5",
  "term_id": "GO:0048306",
  "gene": "UniProtKB:P33763"
}